{
  "term_id": "UNKNOWN:0001",
  "gene_symbol": "GPATCH2",
  "gene": "UniProtKB:Q9NW75",
  "term_label": "Unknown molecular function",
  "gene_name": "G patch domain-containing protein 2"
}